{
  "gene_name": "Plasma membrane calcium-transporting ATPase 4",
  "gene": "UniProtKB:P23634",
  "term_id": "GO:0051480",
  "term_label": "regulation of cytosolic calcium ion concentration",
  "gene_symbol": "ATP2B4"
}